regulation of protein kinase C activity [GO:1900019] (biological process) Also known as: regulation of PKC activity, regulation of PKC Subtypes: GO:1900020 Sources: GOC:TermGenie, GOC:signaling Relationships: is a type of regulation of protein serine/threonine kinase activity [GO:0071900]; regulates diacylglycerol-dependent serine/threonine kinase activity [GO:0004697] Definition: Any process that modulates the frequency, rate or extent of protein kinase C activity.